{
  "gene": "UniProtKB:Q7Z6K3",
  "term_label": "Unknown biological process",
  "gene_name": "Protein prenyltransferase alpha subunit repeat-containing protein 1",
  "term_id": "UNKNOWN:0002",
  "gene_symbol": "PTAR1"
}